{
  "gene": "UniProtKB:P11597",
  "gene_symbol": "CETP",
  "term_id": "GO:0034374",
  "term_label": "low-density lipoprotein particle remodeling",
  "gene_name": "Cholesteryl ester transfer protein"
}